protein depalmitoylation [GO:0002084] (biological process) Sources: GOC:hjd Definition: The removal of palymitoyl groups from a lipoprotein. Relationships: is_a protein deacylation [GO:0035601]; is a type of lipoprotein catabolic process [GO:0042159]; is_a GO:0098734